{
  "gene": "UniProtKB:P35900",
  "term_id": "GO:0005856",
  "gene_symbol": "KRT20",
  "term_label": "cytoskeleton",
  "gene_name": "Keratin, type I cytoskeletal 20"
}